{
  "gene_symbol": "ACOD1",
  "term_label": "aconitate decarboxylase activity",
  "term_id": "GO:0047613",
  "gene": "UniProtKB:A6NK06",
  "gene_name": "Cis-aconitate decarboxylase"
}